{
  "gene": "UniProtKB:Q8N944",
  "gene_symbol": "AMER3",
  "term_id": "GO:0005886",
  "term_label": "plasma membrane",
  "gene_name": "APC membrane recruitment protein 3"
}